positive regulation of protein polyubiquitination [GO:1902916] (biological process) Subtypes: positive regulation of protein K63-linked ubiquitination [GO:1902523], positive regulation of protein K48-linked ubiquitination [GO:1902524], positive regulation of protein linear polyubiquitination [GO:1902530] Definition: Any process that activates or increases the frequency, rate or extent of protein polyubiquitination. References: PMID:23645667 Sources: GOC:TermGenie, GOC:di, GO_REF:0000058 Relationships: is a type of positive regulation of protein ubiquitination [GO:0031398]; is a type of regulation of protein polyubiquitination [GO:1902914]; positively regulates protein polyubiquitination [GO:0000209] Also known as: positive regulation of protein polyubiquitinylation, positive regulation of protein polyubiquitylation, up regulation of protein polyubiquitination, up regulation of protein polyubiquitinylation, up regulation of protein polyubiquitylation, up-regulation of protein polyubiquitination, up-regulation of protein polyubiquitinylation, up-regulation of protein polyubiquitylation, upregulation of protein polyubiquitination, upregulation of protein polyubiquitinylation, upregulation of protein polyubiquitylation, activation of protein polyubiquitination, activation of protein polyubiquitinylation, activation of protein polyubiquitylation, activation of polyubiquitin, positive regulation of polyubiquitin, up regulation of polyubiquitin, up-regulation of polyubiquitin, upregulation of polyubiquitin